{
  "gene_symbol": "CDH26",
  "term_label": "cell morphogenesis",
  "term_id": "GO:0000902",
  "gene": "UniProtKB:Q8IXH8",
  "gene_name": "Cadherin-like protein 26"
}